ATP-dependent topological DNA co-entrapment activity [GO:0061776] (molecular function) Definition: A DNA binding activity in which a protein complex interacts with at least one DNA duplex to encircle the DNA molecules with a loose fitting ring. Also known as: ATP-dependent ring closure activity, topological DNA entrapment activity Relationships: is a type of double-stranded DNA binding [GO:0003690] References: PMID:16179255, PMID:26687354, PMID:27797071, PMID:29358048, PMID:37820734 Sources: GOC:dph, GOC:vw